pantothenate biosynthetic process [GO:0015940] (BP) Definition: The chemical reactions and pathways resulting in the formation of pantothenate, the anion of pantothenic acid. It is a B complex vitamin that is a constituent of coenzyme A and is distributed ubiquitously in foods. Sources: GOC:ai, ISBN:0721662544 Also known as: pantothenate anabolism, pantothenate biosynthesis, pantothenate formation, pantothenate synthesis, vitamin B5 biosynthesis, vitamin B5 biosynthetic process, pantothenate anabolism from 2-oxypantoyl lactone, pantothenate anabolism from valine, pantothenate biosynthesis from 2-oxypantoyl lactone, pantothenate biosynthesis from valine, pantothenate biosynthetic process from 2-dehydropantolactone, pantothenate biosynthetic process from 2-oxypantoyl lactone, pantothenate biosynthetic process from valine, pantothenate formation from 2-oxypantoyl lactone, pantothenate formation from valine, pantothenate synthesis from 2-oxypantoyl lactone, pantothenate synthesis from valine Relationships: is a type of pantothenate metabolic process [GO:0015939]; is a type of water-soluble vitamin biosynthetic process [GO:0042364]; is a type of modified amino acid biosynthetic process [GO:0042398]; is_a amide biosynthetic process [GO:0043604]; is a type of monocarboxylic acid biosynthetic process [GO:0072330]